{
  "term_label": "Unknown biological process",
  "gene_name": "Uncharacterized protein",
  "gene_symbol": "A0A494C176",
  "term_id": "UNKNOWN:0002",
  "gene": "UniProtKB:A0A494C176"
}